{
  "gene_name": "Syntaxin-2",
  "term_label": "SNAP receptor activity",
  "term_id": "GO:0005484",
  "gene_symbol": "STX2",
  "gene": "UniProtKB:P32856"
}